{
  "term_label": "apical plasma membrane",
  "gene_name": "Cystic fibrosis transmembrane conductance regulator",
  "term_id": "GO:0016324",
  "gene": "UniProtKB:P13569",
  "gene_symbol": "CFTR"
}